{
  "term_label": "Unknown molecular function",
  "term_id": "UNKNOWN:0001",
  "gene_symbol": "GPR182",
  "gene": "UniProtKB:O15218",
  "gene_name": "G-protein coupled receptor 182"
}